{
  "gene": "UniProtKB:O95817",
  "term_id": "GO:0016020",
  "gene_symbol": "BAG3",
  "term_label": "membrane",
  "gene_name": "BAG family molecular chaperone regulator 3"
}